histone propionyltransferase activity [GO:0061922] (molecular function) Subtypes: GO:0141002 Relationships: is a type of protein propionyltransferase activity [GO:0061920]; is_a histone modifying activity [GO:0140993] References: PMID:17267393 Definition: Catalysis of the reaction: propionyl-CoA + histone = CoA + propionyl-histone.